{
  "gene_name": "Fibroblast growth factor 9",
  "gene_symbol": "FGF9",
  "gene": "UniProtKB:P31371",
  "term_id": "GO:0005104",
  "term_label": "fibroblast growth factor receptor binding"
}